violaceol I catabolic process [GO:1900589] (BP) Also known as: violaceol I breakdown, violaceol I catabolism, violaceol I degradation Definition: The chemical reactions and pathways resulting in the breakdown of violaceol I. Sources: GOC:TermGenie, GOC:di Relationships: is a type of catechol-containing compound catabolic process [GO:0019614]; is a type of secondary metabolite catabolic process [GO:0090487]; is a type of violaceol I metabolic process [GO:1900588]; is a type of ether catabolic process [GO:1901502]